{
  "gene": "UniProtKB:Q9Y2H8",
  "gene_symbol": "ZNF510",
  "gene_name": "Zinc finger protein 510",
  "term_label": "nucleus",
  "term_id": "GO:0005634"
}